{
  "gene": "UniProtKB:P08514",
  "gene_symbol": "ITGA2B",
  "term_label": "integrin alphaIIb-beta3 complex",
  "term_id": "GO:0070442",
  "gene_name": "Integrin alpha-IIb"
}